nucleoside phosphotransferase activity [GO:0050146] (MF) Sources: EC:2.7.1.77, MetaCyc:NUCLEOSIDE-PHOSPHOTRANSFERASE-RXN Definition: Catalysis of the reaction: a nucleotide + a 2'-deoxynucleoside = a nucleoside + a 2'-deoxynucleoside 5'-monophosphate. Also known as: nonspecific nucleoside phosphotransferase activity, nucleotide:2'-nucleoside 5'-phosphotransferase activity, nucleotide:3'-deoxynucleoside 5'-phosphotransferase activity, nucleotide:nucleoside 5'-phosphotransferase activity Relationships: is_a phosphotransferase activity, alcohol group as acceptor [GO:0016773]; is a type of nucleobase-containing compound kinase activity [GO:0019205]